{
  "gene": "UniProtKB:O43292",
  "term_id": "GO:0042765",
  "term_label": "GPI-anchor transamidase complex",
  "gene_name": "Glycosylphosphatidylinositol anchor attachment 1 protein",
  "gene_symbol": "GPAA1"
}